{
  "gene": "UniProtKB:Q01546",
  "term_id": "GO:0045109",
  "gene_symbol": "KRT76",
  "term_label": "intermediate filament organization",
  "gene_name": "Keratin, type II cytoskeletal 2 oral"
}